{
  "gene_name": "Thymosin beta-15B",
  "term_id": "GO:0031941",
  "gene": "UniProtKB:P0CG35",
  "term_label": "filamentous actin",
  "gene_symbol": "TMSB15B"
}